phospholipase A1 activity [GO:0008970] (molecular function) Definition: Catalysis of the reaction: a 1,2-diacyl-sn-glycero-3-phosphocholine + H2O = a 2-acyl-sn-glycero-3-phosphocholine + a fatty acid + H+. Sources: RHEA:18689 Also known as: phosphatidylcholine 1-acylhydrolase activity, phosphatidylserine 1-acylhydrolase activity Relationships: is a type of phospholipase activity [GO:0004620]; is a type of carboxylic ester hydrolase activity [GO:0052689]